{
  "gene_name": "Angio-associated migratory cell protein",
  "gene_symbol": "AAMP",
  "term_label": "Unknown cellular component",
  "term_id": "UNKNOWN:0003",
  "gene": "UniProtKB:Q13685"
}